anterior neural plate formation [GO:0090017] (BP) Definition: The formation of anterior end of the flat, thickened layer of ectodermal cells known as the neural plate. Relationships: is a type of anatomical structure formation involved in morphogenesis [GO:0048646]; is part of GO:0021990 Sources: GOC:dph, GOC:sdb_2009, GOC:tb